{
  "term_label": "plasma membrane",
  "gene_name": "Olfactory receptor 6C3",
  "term_id": "GO:0005886",
  "gene": "UniProtKB:Q9NZP0",
  "gene_symbol": "OR6C3"
}